{
  "term_id": "GO:0004088",
  "gene": "UniProtKB:P31327",
  "gene_symbol": "CPS1",
  "term_label": "carbamoyl-phosphate synthase (glutamine-hydrolyzing) activity",
  "gene_name": "Carbamoyl-phosphate synthase [ammonia], mitochondrial"
}